{
  "gene_symbol": "IL9R",
  "term_label": "interleukin-9-mediated signaling pathway",
  "gene": "UniProtKB:Q01113",
  "term_id": "GO:0038113",
  "gene_name": "Interleukin-9 receptor"
}